{
  "term_label": "Unknown biological process",
  "gene_symbol": "A0A8I5QJS6",
  "gene_name": "Uncharacterized protein",
  "gene": "UniProtKB:A0A8I5QJS6",
  "term_id": "UNKNOWN:0002"
}